{
  "gene": "UniProtKB:Q8TE57",
  "gene_symbol": "ADAMTS16",
  "term_label": "extracellular matrix",
  "term_id": "GO:0031012",
  "gene_name": "A disintegrin and metalloproteinase with thrombospondin motifs 16"
}